{
  "gene": "UniProtKB:A0A494BZU2",
  "term_id": "UNKNOWN:0001",
  "term_label": "Unknown molecular function",
  "gene_name": "BLACAT1 overlapping LEMD1 locus",
  "gene_symbol": "BLACAT1"
}